regulation of mRNA binding [GO:1902415] (biological process) Definition: Any process that modulates the frequency, rate or extent of mRNA binding. Subtypes: positive regulation of mRNA binding [GO:1902416] References: PMID:22890846 Sources: GOC:TermGenie, GOC:rb Relationships: is a type of regulation of binding [GO:0051098]; regulates mRNA binding [GO:0003729]